atrichoblast differentiation [GO:0010055] (biological process) Sources: GOC:tb Relationships: is a type of root epidermal cell differentiation [GO:0010053] Definition: The process in which a relatively unspecialized cell acquires the specialized features of an atrichoblast, a root epidermal cell that will not give rise to a root hair.